{
  "term_id": "GO:0000977",
  "term_label": "RNA polymerase II transcription regulatory region sequence-specific DNA binding",
  "gene_name": "LIM_homeobox protein Lhx6",
  "gene": "UniProtKB:Q9UPM6",
  "gene_symbol": "LHX6"
}